{
  "gene": "UniProtKB:Q9BTT6",
  "term_id": "UNKNOWN:0002",
  "gene_symbol": "LRRC1",
  "gene_name": "Leucine-rich repeat-containing protein 1",
  "term_label": "Unknown biological process"
}